tetracenomycin C catabolic process [GO:1901105] (BP) Sources: GOC:TermGenie, GOC:yaf, UniPathway:UPA00174 Also known as: tetracenomycin C breakdown, tetracenomycin C catabolism, tetracenomycin C degradation Definition: The chemical reactions and pathways resulting in the breakdown of tetracenomycin C. Relationships: is_a polyketide catabolic process [GO:0030640]; is a type of ketone catabolic process [GO:0042182]; is a type of alcohol catabolic process [GO:0046164]; is a type of tertiary alcohol metabolic process [GO:1902644]